{
  "term_label": "Unknown cellular component",
  "gene_name": "Chymotrypsinogen B2",
  "gene": "UniProtKB:Q6GPI1",
  "gene_symbol": "CTRB2",
  "term_id": "UNKNOWN:0003"
}